{
  "gene_symbol": "TACC1",
  "gene_name": "Transforming acidic coiled-coil-containing protein 1",
  "term_label": "Unknown molecular function",
  "term_id": "UNKNOWN:0001",
  "gene": "UniProtKB:O75410"
}